{
  "gene_name": "Protein FAM74A1",
  "term_label": "Unknown cellular component",
  "gene_symbol": "FAM74A1",
  "gene": "UniProtKB:Q5RGS3",
  "term_id": "UNKNOWN:0003"
}